{
  "gene_symbol": "KRTAP5-7",
  "term_label": "Unknown molecular function",
  "term_id": "UNKNOWN:0001",
  "gene": "UniProtKB:Q6L8G8",
  "gene_name": "Keratin-associated protein 5-7"
}